{
  "term_label": "lysosomal membrane",
  "term_id": "GO:0005765",
  "gene_name": "Lysosome-associated membrane glycoprotein 1",
  "gene_symbol": "LAMP1",
  "gene": "UniProtKB:P11279"
}